{
  "gene_symbol": "OR56A4",
  "gene_name": "Olfactory receptor 56A4",
  "term_id": "GO:0005886",
  "gene": "UniProtKB:Q8NGH8",
  "term_label": "plasma membrane"
}